regulation of production of molecular mediator of immune response [GO:0002700] (biological process) Relationships: is a type of regulation of immune effector process [GO:0002697]; is a type of regulation of gene expression [GO:0010468]; regulates GO:0002440 Definition: Any process that modulates the frequency, rate, or extent of the production of molecular mediator of immune response. Subtypes: regulation of immunoglobulin production [GO:0002637], negative regulation of production of molecular mediator of immune response [GO:0002701], positive regulation of production of molecular mediator of immune response [GO:0002702], regulation of cytokine production involved in immune response [GO:0002718], regulation of antimicrobial peptide production [GO:0002784], GO:0071661, GO:2000511 Sources: GOC:add